{
  "gene_symbol": "DYDC2",
  "gene": "UniProtKB:Q96IM9",
  "term_id": "UNKNOWN:0001",
  "gene_name": "DPY30 domain-containing protein 2",
  "term_label": "Unknown molecular function"
}